{
  "gene": "UniProtKB:P51168",
  "term_label": "plasma membrane",
  "term_id": "GO:0005886",
  "gene_name": "Amiloride-sensitive sodium channel subunit beta",
  "gene_symbol": "SCNN1B"
}